exoribonuclease H activity [GO:0004533] (molecular function) Also known as: retroviral reverse transcriptase RNaseH Definition: Catalysis of the exonucleolytic cleavage of RNA to 5'-phosphomonoester oligonucleotides in both 5' to 3' and 3' to 5' directions. Sources: EC:3.1.13.2 Relationships: is_a RNA exonuclease activity, producing 5'-phosphomonoesters [GO:0016896]